ferrichrome transmembrane transporter activity [GO:0042929] (MF) Sources: GOC:jl, ISBN:0198506732 Definition: Enables the directed movement of a ferrichrome from one side of a membrane to the other. Ferrichromes are any of a group of growth-promoting Fe(III) chelates formed by various genera of microfungi. They are homodetic cyclic hexapeptides made up of a tripeptide of glycine (or other small neutral amino acids) and a tripeptide of an N'acyl-N4-hydroxy-L-ornithine. Relationships: is a type of siderophore-iron transmembrane transporter activity [GO:0015343]; is a type of amide transmembrane transporter activity [GO:0042887]; BFO_0000050 ferrichrome import into cell [GO:0042928] Also known as: ferrichrome transporter activity